{
  "gene_symbol": "BBS9",
  "gene": "UniProtKB:Q3SYG4",
  "term_label": "cilium assembly",
  "gene_name": "Protein PTHB1",
  "term_id": "GO:0060271"
}